cell wall mannoprotein biosynthetic process [GO:0000032] (biological process) Definition: The chemical reactions and pathways resulting in the formation of cell wall mannoproteins, any cell wall protein that contains covalently bound mannose residues. Relationships: is a type of cell wall glycoprotein biosynthetic process [GO:0031506] Sources: GOC:ai Also known as: cell wall mannoprotein anabolism, cell wall mannoprotein biosynthesis, cell wall mannoprotein formation, cell wall mannoprotein synthesis